{
  "gene_name": "E3 SUMO-protein ligase EGR2",
  "term_label": "regulation of transcription by RNA polymerase II",
  "gene": "UniProtKB:P11161",
  "term_id": "GO:0006357",
  "gene_symbol": "EGR2"
}